{
  "term_id": "GO:0016192",
  "term_label": "vesicle-mediated transport",
  "gene_name": "AP-2 complex subunit beta",
  "gene_symbol": "AP2B1",
  "gene": "UniProtKB:P63010"
}